monoamine oxidase activity [GO:0097621] (molecular function) Also known as: amine:oxygen oxidoreductase (deaminating) activity Note: Acts on primary amines, and also on some secondary and tertiary amines. It differs from EC:1.4.3.21, primary amine oxidase as it can oxidize secondary and tertiary amines but not methylamine. Relationships: is a type of oxidoreductase activity, acting on the CH-NH2 group of donors, oxygen as acceptor [GO:0016641] References: PMID:15279562, PMID:16129825 Sources: GOC:pr Definition: Catalysis of the reaction: RCH2NHR' + H2O + O2 = RCHO + R'NH2 + H2O2.